{
  "term_id": "GO:0005739",
  "gene_name": "Methylmalonate-semialdehyde dehydrogenase [acylating], mitochondrial",
  "gene_symbol": "ALDH6A1",
  "term_label": "mitochondrion",
  "gene": "UniProtKB:Q02252"
}